{
  "gene": "UniProtKB:Q9Y5U5",
  "gene_name": "Tumor necrosis factor receptor superfamily member 18",
  "term_id": "UNKNOWN:0001",
  "term_label": "Unknown molecular function",
  "gene_symbol": "TNFRSF18"
}